alkaloid catabolic process [GO:0009822] (biological process) Subtypes: GO:0019504, cocaine catabolic process [GO:0050784], isoquinoline alkaloid catabolic process [GO:0071274], nicotinate catabolic process [GO:1901848], GO:1901868, ecgonone methyl ester catabolic process [GO:1901871] Also known as: alkaloid breakdown, alkaloid catabolism, alkaloid degradation Sources: GOC:lr, ISBN:0122146743 Definition: The chemical reactions and pathways resulting in the breakdown of alkaloids, nitrogen containing natural products not otherwise classified as peptides, nonprotein amino acids, amines, cyanogenic glycosides, glucosinolates, cofactors, phytohormones or primary metabolites (such as purine or pyrimidine bases). Relationships: is a type of catabolic process [GO:0009056]; is a type of GO:0009820